{
  "gene_symbol": "PCDHGB7",
  "gene": "UniProtKB:Q9Y5F8",
  "term_id": "GO:0007155",
  "term_label": "cell adhesion",
  "gene_name": "Protocadherin gamma-B7"
}